xylulose catabolic process [GO:0005998] (biological process) Relationships: is a type of xylulose metabolic process [GO:0005997]; is a type of pentose catabolic process [GO:0019323] Definition: The chemical reactions and pathways resulting in the breakdown of xylulose, the ketopentose threo-2-pentulose. Sources: ISBN:0198547684 Also known as: xylulose breakdown, xylulose catabolism, xylulose degradation